{
  "gene": "UniProtKB:Q5T0W9",
  "term_label": "signal transduction",
  "gene_symbol": "FAM83B",
  "term_id": "GO:0007165",
  "gene_name": "Protein FAM83B"
}